{
  "gene_symbol": "SUCNR1",
  "gene_name": "Succinate receptor 1",
  "term_label": "plasma membrane",
  "gene": "UniProtKB:Q9BXA5",
  "term_id": "GO:0005886"
}